{
  "term_id": "GO:0006623",
  "term_label": "protein targeting to vacuole",
  "gene": "UniProtKB:Q5THJ4",
  "gene_name": "Intermembrane lipid transfer protein VPS13D",
  "gene_symbol": "VPS13D"
}